nuclear DNA replication factor C complex [GO:0043599] (cellular component) Definition: A nuclear complex of five polypeptides that loads the DNA polymerase processivity factor proliferating cell nuclear antigen (PCNA) onto DNA, thereby permitting processive DNA synthesis catalyzed by DNA polymerase delta or epsilon. In Saccharomyces and several other species, the subunits are known as Rfc1p-Rfc5p, although subunit names do not necessarily correspond between different species. Also known as: nuclear RFC References: PMID:14614842 Sources: GOC:mtg_sensu Relationships: is a type of DNA replication factor C complex [GO:0005663]; is a type of GO:0140513; is part of nuclear replisome [GO:0043601]